{
  "term_label": "phosphatidylinositol-4,5-bisphosphate binding",
  "gene_name": "Gasdermin-C",
  "term_id": "GO:0005546",
  "gene": "UniProtKB:Q9BYG8",
  "gene_symbol": "GSDMC"
}